G protein-coupled neurotransmitter receptor activity involved in regulation of presynaptic membrane potential [GO:0150047] (molecular function) Relationships: is a type of G protein-coupled neurotransmitter receptor activity [GO:0099528]; is part of regulation of presynaptic membrane potential [GO:0099505]; BFO_0000066 GO:0042734 References: PMID:11498050 Sources: GOC:aruk, GOC:bc Definition: G protein-coupled neurotransmitter receptor activity, occurring in the presynaptic membrane, involved in regulation of presynaptic membrane potential. Also known as: G-protein coupled neurotransmitter receptor activity involved in regulation of presynaptic membrane potential